positive regulation of MAP kinase activity [GO:0043406] (biological process) Relationships: is a type of regulation of MAP kinase activity [GO:0043405]; is a type of positive regulation of MAPK cascade [GO:0043410]; is a type of positive regulation of protein serine/threonine kinase activity [GO:0071902]; positively regulates GO:0004707 Sources: GOC:dph, GOC:go_curators Also known as: positive regulation of mitogen activated protein kinase activity, positive regulation of mitogen-activated protein kinase activity, up regulation of MAPK activity, up-regulation of MAPK activity, upregulation of MAPK activity, stimulation of MAPK activity Subtypes: positive regulation of JUN kinase activity [GO:0043507] Definition: Any process that activates or increases the frequency, rate or extent of MAP kinase activity.